{
  "term_label": "sarcomere organization",
  "gene_symbol": "TNNT1",
  "gene_name": "Troponin T, slow skeletal muscle",
  "term_id": "GO:0045214",
  "gene": "UniProtKB:P13805"
}